{
  "term_id": "GO:0005737",
  "term_label": "cytoplasm",
  "gene": "UniProtKB:Q9UMX2",
  "gene_symbol": "OAZ3",
  "gene_name": "Ornithine decarboxylase antizyme 3"
}